{
  "gene": "UniProtKB:Q5JVG8",
  "term_id": "GO:0000978",
  "term_label": "RNA polymerase II cis-regulatory region sequence-specific DNA binding",
  "gene_name": "Zinc finger protein 506",
  "gene_symbol": "ZNF506"
}